{
  "term_label": "nucleus",
  "term_id": "GO:0005634",
  "gene": "UniProtKB:Q9BYG5",
  "gene_name": "Partitioning defective 6 homolog beta",
  "gene_symbol": "PARD6B"
}